{
  "gene_name": "Hemoglobin subunit epsilon",
  "gene_symbol": "HBE1",
  "gene": "UniProtKB:P02100",
  "term_label": "oxygen carrier activity",
  "term_id": "GO:0005344"
}